{
  "gene_name": "Metastasis-associated protein MTA2",
  "term_label": "transcription coactivator activity",
  "gene_symbol": "MTA2",
  "term_id": "GO:0003713",
  "gene": "UniProtKB:O94776"
}